{
  "gene_name": "Zinc finger protein 746",
  "term_id": "GO:0001227",
  "term_label": "DNA-binding transcription repressor activity, RNA polymerase II-specific",
  "gene_symbol": "ZNF746",
  "gene": "UniProtKB:Q6NUN9"
}